{
  "term_label": "disruption of plasma membrane integrity in another organism",
  "gene_symbol": "DEFA5",
  "term_id": "GO:0051673",
  "gene": "UniProtKB:Q01523",
  "gene_name": "Defensin alpha 5"
}